calcineurin-NFAT signaling cascade [GO:0033173] (biological process) Definition: Any intracellular signal transduction in which the signal is passed on within the cell by activation of a member of the NFAT protein family as a consequence of NFAT dephosphorylation by Ca(2+)-activated calcineurin. The cascade begins with calcium-dependent activation of the phosphatase calcineurin. Calcineurin dephosphorylates multiple phosphoserine residues on NFAT, resulting in the translocation of NFAT to the nucleus. The cascade ends with regulation of transcription by NFAT. The calcineurin-NFAT cascade lies downstream of many cell surface receptors, including G protein-coupled receptors (GPCRs) and receptor tyrosine kinases (RTKs) that signal to mobilize calcium ions (Ca2+). Relationships: is a type of calcineurin-mediated signaling [GO:0097720] Regulation: regulated by regulation of calcineurin-NFAT signaling cascade [GO:0070884]; negatively regulated by negative regulation of calcineurin-NFAT signaling cascade [GO:0070885]; positively regulated by positive regulation of calcineurin-NFAT signaling cascade [GO:0070886] References: PMID:12975316, PMID:15928679 Sources: GOC:lm, GOC:mah Also known as: calcineurin-NFAT signaling pathway, calcineurin-NFAT signalling pathway